sterol transmembrane transport [GO:0035382] (BP) Definition: The process in which a sterol is transported across a membrane. Sterols are steroids with one or more hydroxyl groups and a hydrocarbon side-chain in the molecule. Sources: GOC:vw Also known as: sterol membrane transport Note: Note that this term is not intended for use in annotating lateral movement within membranes. Relationships: is_a sterol transport [GO:0015918]; is a type of GO:0055085